{
  "gene_name": "Immunoglobulin superfamily DCC subclass member 3",
  "gene_symbol": "IGDCC3",
  "term_id": "UNKNOWN:0003",
  "term_label": "Unknown cellular component",
  "gene": "UniProtKB:Q8IVU1"
}